negative regulation of telium development [GO:0075278] (biological process) Definition: Any process that stops, prevents, or reduces the frequency, rate or extent of telium development, a process that leads to the formation of a teliospore-bearing sorus of the rust fungi. Sources: GOC:pamgo_curators Relationships: is a type of GO:0075262; is a type of regulation of telium development [GO:0075276]; negatively regulates telium development [GO:0075275]